regulation of metula development [GO:0070802] (biological process) Subtypes: negative regulation of metula development [GO:0070803], positive regulation of metula development [GO:0070804] Sources: GOC:mah Definition: Any process that modulates the frequency, rate or extent of metula development, a process that leads to the formation of metulae. Metulae are elongated mononucleate cells that bud from the surface of the conidiophore tip. Relationships: is a type of regulation of cell development [GO:0060284]; is a type of regulation of conidiophore development [GO:0070793]; regulates metula development [GO:0070789]